{
  "term_id": "GO:0006413",
  "gene_name": "Eukaryotic translation initiation factor 3 subunit E",
  "gene_symbol": "EIF3E",
  "term_label": "translational initiation",
  "gene": "UniProtKB:P60228"
}